neutrophil activation [GO:0042119] (biological process) Regulation: regulated by regulation of neutrophil activation [GO:1902563]; negatively regulated by GO:1902564; positively regulated by positive regulation of neutrophil activation [GO:1902565] Definition: The change in morphology and behavior of a neutrophil resulting from exposure to a cytokine, chemokine, cellular ligand, or soluble factor. Relationships: is a type of GO:0036230 Sources: GOC:mgi_curators, ISBN:0781735149 Subtypes: neutrophil activation involved in immune response [GO:0002283]